{
  "gene_symbol": "CD300LG",
  "gene_name": "CMRF35-like molecule 9",
  "gene": "UniProtKB:Q6UXG3",
  "term_label": "signal transduction",
  "term_id": "GO:0007165"
}